{
  "gene": "UniProtKB:P51841",
  "gene_name": "Retinal guanylyl cyclase 2",
  "term_id": "GO:0007168",
  "term_label": "receptor guanylyl cyclase signaling pathway",
  "gene_symbol": "GUCY2F"
}